{
  "gene_symbol": "PRDM12",
  "gene": "UniProtKB:Q9H4Q4",
  "term_id": "GO:1990226",
  "term_label": "histone methyltransferase binding",
  "gene_name": "PR domain zinc finger protein 12"
}